blood vessel endothelial cell fate specification [GO:0097101] (biological process) Definition: The process involved in the specification of identity of a blood vessel endothelial cell. Once specification has taken place, a cell will be committed to differentiate down a specific pathway if left in its normal environment. A blood vessel endothelial cell is an endothelial cell of the vascular tree, which includes blood vessels and lymphatic vessels. References: PMID:21521739 Sources: CL:0002139, GOC:dgh Relationships: is_a endothelial cell fate specification [GO:0060847]; is part of blood vessel endothelial cell fate commitment [GO:0060846] Subtypes: endothelial tip cell fate specification [GO:0097102], endothelial stalk cell fate specification [GO:0097103]